limonene monooxygenase activity [GO:0019113] (MF) Sources: GOC:mah Definition: Catalysis of a monooxygenase reaction in which oxygen is incorporated into limonene. Relationships: is a type of monooxygenase activity [GO:0004497] Subtypes: (S)-limonene 3-monooxygenase activity [GO:0018674], (S)-limonene 6-monooxygenase activity [GO:0018675], (S)-limonene 7-monooxygenase activity [GO:0018676], GO:0052601, GO:0052741